{
  "term_label": "DNA-binding transcription factor activity",
  "gene": "UniProtKB:Q86WP2",
  "gene_symbol": "GPBP1",
  "term_id": "GO:0003700",
  "gene_name": "Vasculin"
}